{
  "term_id": "UNKNOWN:0003",
  "gene_name": "Immunoglobulin heavy variable 3-72",
  "gene": "UniProtKB:A0A0B4J1Y9",
  "gene_symbol": "IGHV3-72",
  "term_label": "Unknown cellular component"
}